{
  "gene": "UniProtKB:Q07157",
  "gene_symbol": "TJP1",
  "term_label": "positive regulation of blood-brain barrier permeability",
  "term_id": "GO:1905605",
  "gene_name": "Tight junction protein ZO-1"
}